{
  "gene": "UniProtKB:A7E2U8",
  "gene_symbol": "C4orf47",
  "term_label": "Unknown biological process",
  "term_id": "UNKNOWN:0002",
  "gene_name": "UPF0602 protein C4orf47"
}